{
  "term_label": "regulation of transcription by RNA polymerase II",
  "gene": "UniProtKB:P13056",
  "gene_name": "Nuclear receptor subfamily 2 group C member 1",
  "gene_symbol": "NR2C1",
  "term_id": "GO:0006357"
}